{
  "gene_name": "Corticoliberin",
  "gene": "UniProtKB:P06850",
  "gene_symbol": "CRH",
  "term_id": "GO:0017045",
  "term_label": "corticotropin-releasing hormone activity"
}